positive regulation of sterigmatocystin biosynthetic process [GO:0010914] (biological process) Sources: GOC:dph, GOC:tb Definition: Any process that increases the rate, frequency, or extent of sterigmatocystin biosynthesis. Sterigmatocystin biosynthetic processes are the chemical reactions and pathways resulting in the formation of sterigmatocystin, a carcinogenic mycotoxin produced in high yields by strains of the common molds. Relationships: is a type of regulation of sterigmatocystin biosynthetic process [GO:0010913]; is a type of positive regulation of secondary metabolite biosynthetic process [GO:1900378]; positively regulates sterigmatocystin biosynthetic process [GO:0045461]